{
  "term_label": "Unknown biological process",
  "gene_symbol": "MUC3A",
  "gene": "UniProtKB:Q02505",
  "term_id": "UNKNOWN:0002",
  "gene_name": "Mucin-3A"
}